{
  "gene_name": "Protein HIDE1",
  "term_id": "UNKNOWN:0001",
  "gene": "UniProtKB:A8MVS5",
  "gene_symbol": "HIDE1",
  "term_label": "Unknown molecular function"
}